{
  "term_id": "GO:0043525",
  "gene": "UniProtKB:Q07820",
  "gene_symbol": "MCL1",
  "term_label": "positive regulation of neuron apoptotic process",
  "gene_name": "Induced myeloid leukemia cell differentiation protein Mcl-1"
}